glyceraldehyde-3-phosphate dehydrogenase (ferredoxin) activity [GO:0043797] (molecular function) Also known as: D-glyceraldehyde-3-phosphate:ferredoxin oxidoreductase activity, GAPOR, glyceraldehyde-3-phosphate Fd oxidoreductase activity, glyceraldehyde-3-phosphate ferredoxin reductase activity Relationships: is a type of oxidoreductase activity, acting on the aldehyde or oxo group of donors, iron-sulfur protein as acceptor [GO:0016625] References: PMID:11265456, PMID:7721730 Sources: RHEA:24148 Definition: Catalysis of the reaction: D-glyceraldehyde-3-phosphate + H2O + 2 oxidized ferredoxin = 3-phospho-D-glycerate + 2 H+ + 2 reduced ferredoxin.